{
  "gene_name": "Protein shisa-8",
  "gene_symbol": "SHISA8",
  "term_label": "Unknown molecular function",
  "term_id": "UNKNOWN:0001",
  "gene": "UniProtKB:B8ZZ34"
}